{
  "term_label": "5'-nucleotidase activity",
  "gene": "UniProtKB:Q5TFE4",
  "gene_symbol": "NT5DC1",
  "term_id": "GO:0008253",
  "gene_name": "5'-nucleotidase domain-containing protein 1"
}